type 2 mitophagy [GO:0061734] (biological process) Definition: The selective autophagy process in which a mitochondrion is degraded by macroautophagy in a process initiated by mitochondrial depolarization (mtDepo) followed by Parkin binding, and ubiquitination of outer membrane proteins, to remove potentially harm-inducing dysfunctional/damaged mitochondria. Relationships: is a type of GO:0000423 References: PMID:25009776, PMID:25349190 Sources: GOC:vw Also known as: PRKN-mediated mitophagy in response to mitochondrial depolarization, Park2-mediated mitophagy in response to mitochondrial depolarization, parkin-mediated mitophagy in response to mitochondrial depolarization Regulation: regulated by regulation of type 2 mitophagy [GO:1905089]; negatively regulated by negative regulation of type 2 mitophagy [GO:1905090]; positively regulated by GO:1905091